{
  "term_id": "GO:0004177",
  "gene_symbol": "XPNPEP3",
  "gene": "UniProtKB:Q9NQH7",
  "term_label": "aminopeptidase activity",
  "gene_name": "Xaa-Pro aminopeptidase 3"
}